cellular process involved in reproduction in multicellular organism [GO:0022412] (biological process) Relationships: is a type of cellular process [GO:0009987]; is_a GO:0048609 Subtypes: acrosome assembly [GO:0001675], membrane fusion involved in acrosome reaction [GO:0002078], germ cell development [GO:0007281], egg chorion assembly [GO:0007306], eggshell chorion gene amplification [GO:0007307], GO:0007342, cell wall modification involved in fruit ripening [GO:0009829], germline ring canal formation [GO:0030725], sperm plasma membrane disassembly [GO:0035045], egg coat formation [GO:0035803], progesterone secretion [GO:0042701], stromal-epithelial cell signaling involved in prostate gland development [GO:0044345], fusome organization [GO:0045478], GO:0048240, spermatid differentiation [GO:0048515], fusion of sperm to egg plasma membrane involved in double fertilization forming two zygotes [GO:0061935], GO:0061936, stomium development [GO:0080166], GO:0080173, seed trichome differentiation [GO:0090376], seed trichome initiation [GO:0090377], seed trichome elongation [GO:0090378], seed trichome maturation [GO:0090380] Definition: A process, occurring at the cellular level, that is involved in the reproductive function of a multicellular organism. Also known as: reproductive cellular process in multicellular organism Sources: GOC:isa_complete